{
  "term_label": "microvillus",
  "gene_symbol": "MSN",
  "term_id": "GO:0005902",
  "gene_name": "Moesin",
  "gene": "UniProtKB:P26038"
}